{
  "gene_symbol": "DGKK",
  "gene_name": "Diacylglycerol kinase kappa",
  "gene": "UniProtKB:Q5KSL6",
  "term_label": "phosphatidic acid biosynthetic process",
  "term_id": "GO:0006654"
}